{
  "gene_name": "E3 ubiquitin-protein ligase RNF26",
  "gene_symbol": "RNF26",
  "term_label": "Unknown cellular component",
  "term_id": "UNKNOWN:0003",
  "gene": "UniProtKB:Q9BY78"
}